{
  "gene_name": "Pleckstrin homology-like domain family A member 3",
  "term_label": "intrinsic apoptotic signaling pathway in response to DNA damage by p53 class mediator",
  "gene": "UniProtKB:Q9Y5J5",
  "term_id": "GO:0042771",
  "gene_symbol": "PHLDA3"
}